m-AAA complex [GO:0005745] (cellular component) Relationships: is a type of GO:0098800; is a type of peptidase complex [GO:1905368] Definition: Protease complex of the mitochondrial inner membrane that is involved in mitochondrial protein turnover and in processing of proteins imported into mitochondria. References: PMID:12417197, PMID:21147776 Sources: GOC:mcc